{
  "term_id": "GO:0071735",
  "gene_symbol": "IGLC6",
  "term_label": "IgG immunoglobulin complex",
  "gene": "UniProtKB:P0CF74",
  "gene_name": "Immunoglobulin lambda constant 6"
}